endosome to lysosome transport of low-density lipoprotein particle [GO:0090117] (biological process) Also known as: endosome to lysosome transport of LDL Relationships: is a type of endosome to lysosome transport [GO:0008333]; is a type of vesicle-mediated cholesterol transport [GO:0090119] Sources: GOC:ascb_2009, GOC:dph, GOC:tb Definition: The directed movement of low-density lipoprotein particle from endosomes to lysosomes.